{
  "term_label": "glucuronosyltransferase activity",
  "term_id": "GO:0015020",
  "gene_symbol": "UGT2B28",
  "gene": "UniProtKB:Q9BY64",
  "gene_name": "UDP-glucuronosyltransferase 2B28"
}